{
  "gene": "UniProtKB:Q8N5B7",
  "term_label": "endoplasmic reticulum",
  "term_id": "GO:0005783",
  "gene_symbol": "CERS5",
  "gene_name": "Ceramide synthase 5"
}